{
  "gene_symbol": "SMRP1",
  "gene": "UniProtKB:Q8NCR6",
  "term_id": "GO:0043014",
  "gene_name": "Spermatid-specific manchette-related protein 1",
  "term_label": "alpha-tubulin binding"
}